{
  "gene_symbol": "ZNF347",
  "gene": "UniProtKB:Q96SE7",
  "term_label": "RNA polymerase II cis-regulatory region sequence-specific DNA binding",
  "gene_name": "Zinc finger protein 347",
  "term_id": "GO:0000978"
}